{
  "gene_symbol": "SERPINB10",
  "term_label": "Unknown biological process",
  "gene_name": "Serpin B10",
  "gene": "UniProtKB:P48595",
  "term_id": "UNKNOWN:0002"
}